endoribonuclease inhibitor activity [GO:0060698] (molecular function) Relationships: is a type of ribonuclease inhibitor activity [GO:0008428]; negatively regulates RNA endonuclease activity [GO:0004521] Definition: Binds to and stops, prevents or reduces the activity of endoribonuclease. Sources: GOC:dph, GOC:tb